{
  "term_id": "GO:0046854",
  "gene": "UniProtKB:Q86TV6",
  "gene_symbol": "TTC7B",
  "term_label": "phosphatidylinositol phosphate biosynthetic process",
  "gene_name": "Tetratricopeptide repeat protein 7B"
}